{
  "term_id": "GO:0019221",
  "gene_name": "Growth hormone receptor",
  "gene": "UniProtKB:P10912",
  "gene_symbol": "GHR",
  "term_label": "cytokine-mediated signaling pathway"
}